organelle fission [GO:0048285] (biological process) Sources: GOC:jid Definition: The creation of two or more organelles by division of one organelle. Relationships: is a type of organelle organization [GO:0006996] Subtypes: mitochondrial fission [GO:0000266], nuclear division [GO:0000280], peroxisome fission [GO:0016559], plastid fission [GO:0043572], GO:0140285, vacuole fission [GO:0140572], lysosome fission [GO:0170064]